{
  "gene_symbol": "GALNT8",
  "term_id": "GO:0004653",
  "term_label": "polypeptide N-acetylgalactosaminyltransferase activity",
  "gene_name": "Probable polypeptide N-acetylgalactosaminyltransferase 8",
  "gene": "UniProtKB:Q9NY28"
}